digestive system development [GO:0055123] (biological process) Sources: GOC:jid Definition: The process whose specific outcome is the progression of the digestive system over time, from its formation to the mature structure. The digestive system is the entire structure in which digestion takes place. Digestion is all of the physical, chemical, and biochemical processes carried out by multicellular organisms to break down ingested nutrients into components that may be easily absorbed and directed into metabolism. Relationships: is a type of system development [GO:0048731]